{
  "gene": "UniProtKB:Q0VDD7",
  "term_label": "Unknown molecular function",
  "gene_name": "Break repair meiotic recombinase recruitment factor 1",
  "term_id": "UNKNOWN:0001",
  "gene_symbol": "BRME1"
}